{
  "term_label": "nucleus",
  "gene": "UniProtKB:Q9ULM2",
  "gene_symbol": "ZNF490",
  "gene_name": "Zinc finger protein 490",
  "term_id": "GO:0005634"
}